{
  "gene": "UniProtKB:Q569K4",
  "gene_name": "Zinc finger protein 385B",
  "gene_symbol": "ZNF385B",
  "term_id": "UNKNOWN:0002",
  "term_label": "Unknown biological process"
}